{
  "gene_symbol": "XAF1",
  "gene_name": "XIAP-associated factor 1",
  "term_label": "mitochondrion",
  "gene": "UniProtKB:Q6GPH4",
  "term_id": "GO:0005739"
}